endothelial cell-cell adhesion [GO:0071603] (biological process) Definition: The attachment of an endothelial cell to another endothelial cell via adhesion molecules. Relationships: is a type of epithelial cell-cell adhesion [GO:0090136] Sources: GOC:BHF